{
  "gene_symbol": "AURKC",
  "gene": "UniProtKB:Q9UQB9",
  "gene_name": "Aurora kinase C",
  "term_label": "spindle pole",
  "term_id": "GO:0000922"
}